{
  "gene": "UniProtKB:Q9H2G2",
  "term_id": "GO:0004674",
  "gene_symbol": "SLK",
  "term_label": "protein serine/threonine kinase activity",
  "gene_name": "STE20-like serine_threonine-protein kinase"
}